L-amino acid transmembrane transporter activity [GO:0015179] (molecular function) Definition: Enables the transfer of an L-amino acid from one side of a membrane to the other. L-amino acids are the L-enantiomers of amino acids. Sources: GOC:ai, GOC:jsg, GOC:mah, GOC:mtg_transport, ISBN:0815340729 Also known as: L-amino acid transporter activity Relationships: is a type of amino acid transmembrane transporter activity [GO:0015171]; is a type of carboxylic acid transmembrane transporter activity [GO:0046943]; BFO_0000050 L-alpha-amino acid transmembrane transport [GO:1902475] Subtypes: L-ornithine transmembrane transporter activity [GO:0000064], 3-sulfino-L-alanine: proton, glutamate antiporter activity [GO:0000514], GO:0005290, GO:0005302, L-valine transmembrane transporter activity [GO:0005304], GO:0005313, L-alanine transmembrane transporter activity [GO:0015180], L-asparagine transmembrane transporter activity [GO:0015182], L-aspartate transmembrane transporter activity [GO:0015183], L-cystine transmembrane transporter activity [GO:0015184], L-glutamine transmembrane transporter activity [GO:0015186], L-isoleucine transmembrane transporter activity [GO:0015188], GO:0015189, L-leucine transmembrane transporter activity [GO:0015190], L-methionine transmembrane transporter activity [GO:0015191], L-phenylalanine transmembrane transporter activity [GO:0015192], L-proline transmembrane transporter activity [GO:0015193], GO:0015194, L-threonine transmembrane transporter activity [GO:0015195], L-tryptophan transmembrane transporter activity [GO:0015196], GO:0015626, GO:0034590, L-amino acid efflux transmembrane transporter activity [GO:0034639], GO:0042970, L-arginine transmembrane transporter activity [GO:0061459], L-kynurenine transmembrane transporter activity [GO:0140926], S-adenosyl-L-methionine:S-adenosyl-L-homocysteine antiporter activity [GO:0180003]